response to steroid hormone [GO:0048545] (biological process) Also known as: response to steroid hormone stimulus Sources: GOC:go_curators Subtypes: GO:0031960, response to progesterone [GO:0032570], GO:0051467, cellular response to steroid hormone stimulus [GO:0071383] Relationships: is a type of response to hormone [GO:0009725]; is a type of GO:0033993 Definition: Any process that results in a change in state or activity of a cell or an organism (in terms of movement, secretion, enzyme production, gene expression, etc.) as a result of a steroid hormone stimulus.